{
  "gene_symbol": "MTMR1",
  "term_id": "GO:0005737",
  "gene_name": "Myotubularin-related protein 1",
  "gene": "UniProtKB:Q13613",
  "term_label": "cytoplasm"
}